{
  "term_label": "ubiquitin-like ligase-substrate adaptor activity",
  "gene_symbol": "IPP",
  "term_id": "GO:1990756",
  "gene_name": "Actin-binding protein IPP",
  "gene": "UniProtKB:Q9Y573"
}